{
  "gene_symbol": "PRR23D1",
  "gene": "UniProtKB:E9PI22",
  "gene_name": "Proline-rich protein 23D1",
  "term_label": "Unknown biological process",
  "term_id": "UNKNOWN:0002"
}